{
  "gene_name": "Taste receptor type 2 member 41",
  "gene_symbol": "TAS2R41",
  "term_id": "UNKNOWN:0002",
  "gene": "UniProtKB:P59536",
  "term_label": "Unknown biological process"
}